response to 3,3',4,4',5-pentachlorobiphenyl [GO:1904610] (biological process) Definition: Any process that results in a change in state or activity of a cell or an organism (in terms of movement, secretion, enzyme production, gene expression, etc.) as a result of a 3,3',4,4',5-pentachlorobiphenyl stimulus. Subtypes: cellular response to 3,3',4,4',5-pentachlorobiphenyl [GO:1904611] Also known as: response to PCB 126 References: PMID:23196670 Sources: GOC:TermGenie, GO_REF:0000071 Relationships: is a type of response to chemical [GO:0042221]